{
  "gene": "UniProtKB:O15467",
  "gene_symbol": "CCL16",
  "term_label": "eosinophil chemotaxis",
  "gene_name": "C-C motif chemokine 16",
  "term_id": "GO:0048245"
}